{
  "gene_symbol": "MPPE1",
  "term_id": "UNKNOWN:0001",
  "gene": "UniProtKB:Q53F39",
  "gene_name": "Metallophosphoesterase 1",
  "term_label": "Unknown molecular function"
}